{
  "gene": "UniProtKB:P0DSO1",
  "gene_symbol": "FAM246C",
  "term_label": "Unknown cellular component",
  "gene_name": "Protein FAM246C",
  "term_id": "UNKNOWN:0003"
}